response to red light [GO:0010114] (biological process) Definition: Any process that results in a change in state or activity of a cell or an organism (in terms of movement, secretion, enzyme production, gene expression, etc.) as a result of a red light stimulus. Red light is electromagnetic radiation of wavelength of 580-700nm. An example of this response is seen at the beginning of many plant species developmental stages. These include germination, and the point when cotyledon expansion is triggered. In certain species these processes take place in response to absorption of red light by the pigment molecule phytochrome, but the signal can be reversed by exposure to far red light. During the initial phase the phytochrome molecule is only present in the red light absorbing form, but on absorption of red light it changes to a far red light absorbing form, triggering progress through development. An immediate short period of exposure to far red light entirely returns the pigment to its initial state and prevents triggering of the developmental process. A thirty minute break between red and subsequent far red light exposure renders the red light effect irreversible, and development then occurs regardless of whether far red light exposure subsequently occurs. Also known as: response to red light stimulus Subtypes: GO:0009907, response to low fluence red light stimulus [GO:0010202], GO:0010203, cellular response to red light [GO:0071491] Sources: GOC:mtg_far_red, GOC:sm Relationships: is a type of response to red or far red light [GO:0009639]